{
  "gene": "UniProtKB:Q14249",
  "gene_symbol": "ENDOG",
  "gene_name": "Endonuclease G, mitochondrial",
  "term_label": "mitochondrial inner membrane",
  "term_id": "GO:0005743"
}